{
  "term_id": "GO:0006955",
  "gene": "UniProtKB:A0A075B6H7",
  "gene_name": "Probable non-functional immunoglobulin kappa variable 3-7",
  "gene_symbol": "IGKV3-7",
  "term_label": "immune response"
}